regulation of monocyte extravasation [GO:2000437] (biological process) Sources: GOC:obol Definition: Any process that modulates the frequency, rate or extent of monocyte extravasation. Subtypes: negative regulation of monocyte extravasation [GO:2000438], positive regulation of monocyte extravasation [GO:2000439] Relationships: is a type of regulation of cellular extravasation [GO:0002691]; is a type of regulation of mononuclear cell migration [GO:0071675]; regulates monocyte extravasation [GO:0035696]